{
  "gene": "UniProtKB:Q9UJG1",
  "gene_symbol": "MOSPD1",
  "gene_name": "Motile sperm domain-containing protein 1",
  "term_label": "Unknown cellular component",
  "term_id": "UNKNOWN:0003"
}